symbiont-mediated perturbation of host phagocytosis [GO:0052067] (biological process) References: PMID:23084912, PMID:29114249 Also known as: modulation by organism of entry into host via host phagocytosis, modulation by symbiont of entry into host via phagocytosis, disruption of host phagocytosis, inhibition by symbiont of entry into host cell via phagocytosis, antiphagocytosis, phagocytosis avoidance Relationships: is a type of symbiont-mediated perturbation of host defenses [GO:0030682] Definition: A process in which in a symbiont interferes with or inhibits host phagocytosis by targeting phagocytic signaling or the cellular phagocytic machinery. The host is defined as the larger of the organisms involved in a symbiotic interaction.